{
  "gene_name": "Cyclin-A1",
  "term_id": "GO:0016538",
  "term_label": "cyclin-dependent protein serine/threonine kinase regulator activity",
  "gene_symbol": "CCNA1",
  "gene": "UniProtKB:P78396"
}